{
  "term_id": "GO:0045271",
  "term_label": "respiratory chain complex I",
  "gene": "UniProtKB:Q9UI09",
  "gene_name": "NADH dehydrogenase [ubiquinone] 1 alpha subcomplex subunit 12",
  "gene_symbol": "NDUFA12"
}